positive regulation of blood vessel endothelial cell differentiation [GO:0110058] (biological process) References: PMID:23072816 Sources: GOC:BHF, GOC:BHF_miRNA, GOC:rph Definition: Any process that activates or increases the frequency, rate or extent of blood vessel endothelial cell differentiation. Relationships: is a type of GO:0045603; is_a GO:0110057; positively regulates blood vessel endothelial cell differentiation [GO:0060837] Subtypes: positive regulation of venous endothelial cell fate commitment [GO:2000789]